macromolecule metabolic process [GO:0043170] (biological process) Relationships: is a type of GO:0008152 Also known as: biopolymer metabolic process, macromolecule metabolism, organismal macromolecule metabolism, multicellular organismal macromolecule metabolic process Subtypes: polysaccharide metabolic process [GO:0005976], aminoglycan metabolic process [GO:0006022], GO:0008653, macromolecule catabolic process [GO:0009057], macromolecule biosynthetic process [GO:0009059], protein metabolic process [GO:0019538], GO:0043112, macromolecule modification [GO:0043412], cell wall macromolecule metabolic process [GO:0044036], GO:0046374, GO:0046375, colanic acid metabolic process [GO:0046377], nucleic acid metabolic process [GO:0090304], polynucleotide 3' dephosphorylation [GO:0098506], GO:0098507, ATP generation from poly-ADP-D-ribose [GO:1990966], amylopectin metabolic process [GO:2000896] Sources: GOC:mah Definition: The chemical reactions and pathways involving macromolecules, any molecule of high relative molecular mass, the structure of which essentially comprises the multiple repetition of units derived, actually or conceptually, from molecules of low relative molecular mass. Regulation: positively regulated by positive regulation of macromolecule metabolic process [GO:0010604]; RO_0002212 by GO:0010605; RO_0002211 by GO:0060255